{
  "term_label": "calcium ion binding",
  "term_id": "GO:0005509",
  "gene_name": "Group IIF secretory phospholipase A2",
  "gene_symbol": "PLA2G2F",
  "gene": "UniProtKB:Q9BZM2"
}